{
  "term_id": "GO:0016020",
  "gene_name": "Neuronal vesicle trafficking-associated protein 2",
  "gene": "UniProtKB:Q9Y328",
  "gene_symbol": "NSG2",
  "term_label": "membrane"
}